{
  "gene_symbol": "SGMS1",
  "term_label": "ceramide cholinephosphotransferase activity",
  "gene_name": "Phosphatidylcholine:ceramide cholinephosphotransferase 1",
  "gene": "UniProtKB:Q86VZ5",
  "term_id": "GO:0047493"
}